{
  "gene_symbol": "MAP2K3",
  "gene": "UniProtKB:P46734",
  "gene_name": "Dual specificity mitogen-activated protein kinase kinase 3",
  "term_label": "Unknown cellular component",
  "term_id": "UNKNOWN:0003"
}